{
  "term_id": "UNKNOWN:0003",
  "gene_symbol": "LRRC63",
  "term_label": "Unknown cellular component",
  "gene": "UniProtKB:Q05C16",
  "gene_name": "Leucine-rich repeat-containing protein 63"
}